{
  "term_id": "GO:0032797",
  "term_label": "SMN complex",
  "gene_symbol": "DDX20",
  "gene": "UniProtKB:Q9UHI6",
  "gene_name": "Probable ATP-dependent RNA helicase DDX20"
}